tungstate binding [GO:1901359] (molecular function) Definition: Binding to tungstate. Relationships: is a type of anion binding [GO:0043168] Sources: GOC:TermGenie